{
  "gene_name": "Homeobox protein goosecoid-2",
  "gene_symbol": "GSC2",
  "term_label": "regulation of transcription by RNA polymerase II",
  "gene": "UniProtKB:O15499",
  "term_id": "GO:0006357"
}